{
  "gene_symbol": "PACSIN1",
  "term_id": "GO:0097320",
  "term_label": "plasma membrane tubulation",
  "gene_name": "Protein kinase C and casein kinase substrate in neurons protein 1",
  "gene": "UniProtKB:Q9BY11"
}